{
  "gene_name": "Class E basic helix-loop-helix protein 41",
  "term_id": "GO:0050767",
  "term_label": "regulation of neurogenesis",
  "gene_symbol": "BHLHE41",
  "gene": "UniProtKB:Q9C0J9"
}